{
  "term_id": "GO:0005634",
  "gene": "UniProtKB:Q6P1L6",
  "gene_name": "Zinc finger protein 343",
  "term_label": "nucleus",
  "gene_symbol": "ZNF343"
}